{
  "gene_symbol": "SMAD5",
  "term_id": "GO:0060395",
  "gene": "UniProtKB:Q99717",
  "term_label": "SMAD protein signal transduction",
  "gene_name": "Mothers against decapentaplegic homolog 5"
}